{
  "gene_name": "Serine_threonine-protein kinase ULK1",
  "gene": "UniProtKB:O75385",
  "gene_symbol": "ULK1",
  "term_id": "GO:0004674",
  "term_label": "protein serine/threonine kinase activity"
}